{
  "gene_name": "Zinc transporter ZIP1",
  "term_label": "zinc ion transmembrane transporter activity",
  "gene": "UniProtKB:Q9NY26",
  "gene_symbol": "SLC39A1",
  "term_id": "GO:0005385"
}